{
  "gene_symbol": "OR56A5",
  "term_label": "Unknown biological process",
  "gene_name": "Olfactory receptor 56A5",
  "term_id": "UNKNOWN:0002",
  "gene": "UniProtKB:P0C7T3"
}